{
  "term_label": "Unknown cellular component",
  "gene_name": "Putative endogenous retrovirus group K member 11-1 Env polyprotein",
  "term_id": "UNKNOWN:0003",
  "gene": "UniProtKB:P61568",
  "gene_symbol": "ERVK11-1"
}